{
  "gene": "UniProtKB:O60729",
  "gene_name": "Dual specificity protein phosphatase CDC14B",
  "gene_symbol": "CDC14B",
  "term_label": "mitotic spindle",
  "term_id": "GO:0072686"
}